{
  "gene_name": "Exocyst complex component 5",
  "term_id": "GO:0006893",
  "gene_symbol": "EXOC5",
  "gene": "UniProtKB:O00471",
  "term_label": "Golgi to plasma membrane transport"
}